protein-phycobiliviolin linkage [GO:0017008] (biological process) Definition: The linkage of the chromophore phycobiliviolin to phycoerythrocyanin. Sources: RESID:AA0258 Relationships: is a type of protein-bilin linkage [GO:0017007]